inner cell mass cell fate commitment [GO:0001827] (biological process) Relationships: is a type of cell fate commitment [GO:0045165]; is part of GO:0001826 Definition: The cell fate commitment of precursor cells that will become inner cell mass cells. Sources: GOC:dph, ISBN:0124020607, ISBN:0198542771 Note: See also the Anatomical Dictionary for Mouse Development ontology terms 'TS4, compacted morula ; EMAP:13' and 'TS4, inner cell mass ; EMAP:14'.